mitochondrion targeting sequence binding [GO:0030943] (molecular function) Relationships: is a type of signal sequence binding [GO:0005048] Sources: GOC:mah Definition: Binding to a mitochondrion targeting sequence, a specific peptide sequence that acts as a signal to localize the protein within the mitochondrion. Also known as: mitochondrial targeting sequence binding